{
  "gene": "UniProtKB:Q9NZI8",
  "gene_name": "Insulin-like growth factor 2 mRNA-binding protein 1",
  "gene_symbol": "IGF2BP1",
  "term_id": "GO:0010494",
  "term_label": "cytoplasmic stress granule"
}